{
  "gene": "UniProtKB:A0A3B3IRS2",
  "term_id": "UNKNOWN:0002",
  "gene_symbol": "LOC647264",
  "gene_name": "Uncharacterized protein",
  "term_label": "Unknown biological process"
}